{
  "gene_name": "Keratin-associated protein 21-1",
  "gene": "UniProtKB:Q3LI58",
  "gene_symbol": "KRTAP21-1",
  "term_id": "UNKNOWN:0001",
  "term_label": "Unknown molecular function"
}